{
  "term_label": "Unknown molecular function",
  "gene_symbol": "RPH3A",
  "term_id": "UNKNOWN:0001",
  "gene": "UniProtKB:Q9Y2J0",
  "gene_name": "Rabphilin-3A"
}